negative regulation of interleukin-18-mediated signaling pathway [GO:2000493] (biological process) Definition: Any process that stops, prevents or reduces the frequency, rate or extent of interleukin-18-mediated signaling pathway. Sources: GOC:obol Relationships: is a type of negative regulation of cytokine-mediated signaling pathway [GO:0001960]; is_a regulation of interleukin-18-mediated signaling pathway [GO:2000492]; negatively regulates GO:0035655 Also known as: negative regulation of interleukin-18-mediated signalling pathway